{
  "term_id": "GO:0042383",
  "term_label": "sarcolemma",
  "gene": "UniProtKB:P32418",
  "gene_name": "Sodium_calcium exchanger 1",
  "gene_symbol": "SLC8A1"
}